positive regulation of gastrin-induced gastric acid secretion [GO:1903641] (biological process) Relationships: is a type of positive regulation of gastric acid secretion [GO:0060454]; is a type of regulation of gastrin-induced gastric acid secretion [GO:1903639]; positively regulates gastrin-induced gastric acid secretion [GO:0001698] Definition: Any process that activates or increases the frequency, rate or extent of gastrin-induced gastric acid secretion. References: PMID:11123201 Sources: GOC:TermGenie, GO_REF:0000058 Also known as: up regulation of gastrin-induced gastric acid secretion, up-regulation of gastrin-induced gastric acid secretion, upregulation of gastrin-induced gastric acid secretion, activation of gastrin-induced gastric acid secretion